amphibian larval development [GO:0002117] (biological process) Definition: The process whose specific outcome is the progression of the amphibian larva over time, from its formation to the mature structure. Amphibian larvae, sometimes called pollywogs or tadpoles, hatch from eggs and begin to grow limbs and other adult physical features at various times, depending on the species, before they metamorphose into the adult form. References: PMID:27143402 Sources: GOC:bf Relationships: is a type of larval development [GO:0002164]